{
  "gene_name": "C-C motif chemokine 26",
  "term_label": "extracellular space",
  "gene": "UniProtKB:Q9Y258",
  "gene_symbol": "CCL26",
  "term_id": "GO:0005615"
}